mitotic spindle astral microtubule [GO:0061673] (cellular component) Definition: Any of the mitotic spindle microtubules that radiate in all directions from the spindle poles and are thought to contribute to the forces that separate the poles and position them in relation to the rest of the cell. Relationships: is a type of astral microtubule [GO:0000235]; is part of GO:0072686 Sources: GOC:dph